{
  "term_id": "GO:0010494",
  "term_label": "cytoplasmic stress granule",
  "gene_symbol": "DDX25",
  "gene": "UniProtKB:Q9UHL0",
  "gene_name": "ATP-dependent RNA helicase DDX25"
}